neurotrophin TRKB receptor binding [GO:0005169] (molecular function) Sources: GOC:ai Relationships: is a type of neurotrophin TRK receptor binding [GO:0005167] Definition: Binding to a neurotrophin TRKB receptor. Also known as: neurotrophin TRKB receptor ligand